hematopoietic or lymphoid organ development [GO:0048534] (BP) Sources: GOC:add, GOC:rl, ISBN:0781735149 Definition: The process whose specific outcome is the progression of any organ involved in hematopoiesis (also known as hemopoiesis) or lymphoid cell activation over time, from its formation to the mature structure. Such development includes differentiation of resident cell types (stromal cells) and of migratory cell types dependent on the unique microenvironment afforded by the organ for their proper differentiation. Relationships: is a type of animal organ development [GO:0048513]; BFO_0000050 immune system development [GO:0002520] Subtypes: GO:0048535, GO:0048536, mucosa-associated lymphoid tissue development [GO:0048537], thymus development [GO:0048538], bone marrow development [GO:0048539], bursa of Fabricius development [GO:0048540], lymph gland development [GO:0048542], head kidney development [GO:0072113] Also known as: haematopoietic or lymphoid organ development, haemopoietic or lymphoid organ development, hemopoietic or lymphoid organ development